{
  "term_id": "GO:0005769",
  "term_label": "early endosome",
  "gene": "UniProtKB:Q5SW96",
  "gene_symbol": "LDLRAP1",
  "gene_name": "Low density lipoprotein receptor adapter protein 1"
}